generative cell mitosis [GO:0055047] (biological process) Sources: GOC:mtg_plant Definition: The process in which the generative cell divides by mitosis to form two haploid cells. These will subsequently differentiate into sperm cells. Relationships: is a type of GO:0140014; is part of GO:0048232